{
  "term_id": "GO:0060271",
  "gene_name": "Meckelin",
  "term_label": "cilium assembly",
  "gene": "UniProtKB:Q5HYA8",
  "gene_symbol": "TMEM67"
}